{
  "term_id": "GO:0006956",
  "term_label": "complement activation",
  "gene": "UniProtKB:Q02985",
  "gene_symbol": "CFHR3",
  "gene_name": "Complement factor H-related protein 3"
}